{
  "gene_symbol": "PHACTR4",
  "gene_name": "Phosphatase and actin regulator 4",
  "term_label": "actin cytoskeleton organization",
  "gene": "UniProtKB:Q8IZ21",
  "term_id": "GO:0030036"
}